{
  "term_label": "membrane",
  "gene": "UniProtKB:Q9NYV9",
  "gene_symbol": "TAS2R13",
  "term_id": "GO:0016020",
  "gene_name": "Taste receptor type 2 member 13"
}